methionine adenosyltransferase activity [GO:0004478] (molecular function) Definition: Catalysis of the reaction: ATP + L-methionine + H2O = phosphate + diphosphate + S-adenosyl-L-methionine. Sources: EC:2.5.1.6 Relationships: is a type of transferase activity, transferring alkyl or aryl (other than methyl) groups [GO:0016765] Regulation: regulated by GO:0048270 Also known as: ATP-methionine adenosyltransferase activity, ATP:L-methionine S-adenosyltransferase activity, AdoMet synthetase activity, S-adenosyl-L-methionine synthetase activity, S-adenosylmethionine synthase activity, S-adenosylmethionine synthetase activity, adenosylmethionine synthetase activity, methionine S-adenosyltransferase activity, methionine-activating enzyme